{
  "gene_symbol": "KLK12",
  "gene_name": "Kallikrein-12",
  "gene": "UniProtKB:Q9UKR0",
  "term_label": "serine-type endopeptidase activity",
  "term_id": "GO:0004252"
}